{
  "gene_name": "Brain mitochondrial carrier protein 1",
  "gene_symbol": "SLC25A14",
  "term_id": "GO:1900407",
  "term_label": "regulation of cellular response to oxidative stress",
  "gene": "UniProtKB:O95258"
}